{
  "gene_symbol": "EDRF1",
  "gene": "UniProtKB:Q3B7T1",
  "gene_name": "Erythroid differentiation-related factor 1",
  "term_label": "Unknown cellular component",
  "term_id": "UNKNOWN:0003"
}